{
  "term_id": "GO:0005737",
  "gene": "UniProtKB:Q5JR98",
  "gene_name": "Dynein light chain Tctex-type 4",
  "term_label": "cytoplasm",
  "gene_symbol": "DYNLT4"
}